{
  "gene_name": "Potassium voltage-gated channel subfamily D member 1",
  "gene": "UniProtKB:Q9NSA2",
  "term_label": "action potential",
  "gene_symbol": "KCND1",
  "term_id": "GO:0001508"
}